{
  "term_label": "nucleus",
  "term_id": "GO:0005634",
  "gene": "UniProtKB:Q96JN0",
  "gene_symbol": "LCOR",
  "gene_name": "Ligand-dependent corepressor"
}